alphaIIb-beta3 integrin-CIB complex [GO:0070769] (cellular component) Also known as: ITGA2B-ITGB3-CIB1 complex Definition: A protein complex that consists of an alphaIIb-beta3 integrin complex bound to CIB, a protein that binds calcium as well as the alphaIIb-beta3 integrin. References: PMID:9030514 Relationships: is a type of plasma membrane protein complex [GO:0098797]